{
  "term_id": "UNKNOWN:0002",
  "gene": "UniProtKB:Q8IWL2",
  "term_label": "Unknown biological process",
  "gene_name": "Pulmonary surfactant-associated protein A1",
  "gene_symbol": "SFTPA1"
}